(R)-mevalonic acid biosynthetic process [GO:1901737] (biological process) Definition: The chemical reactions and pathways resulting in the formation of (R)-mevalonic acid. Sources: GOC:TermGenie, GOC:yaf, UniPathway:UPA00058 Also known as: (R)-mevalonate anabolism, (R)-mevalonate biosynthesis, (R)-mevalonate synthesis, (R)-mevalonic acid anabolism, (R)-mevalonic acid biosynthesis, (R)-mevalonic acid formation, (R)-mevalonic acid synthesis Relationships: is a type of GO:0072330 Regulation: regulated by GO:0106107; negatively regulated by negative regulation of (R)-mevalonic acid biosynthetic process [GO:0106108]; positively regulated by GO:0106109